extrinsic component of plasma membrane [GO:0019897] (cellular component) Also known as: juxtamembrane, extrinsic to plasma membrane, peripheral plasma membrane protein Definition: The component of a plasma membrane consisting of gene products and protein complexes that are loosely bound to one of its surfaces, but not integrated into the hydrophobic region. Subtypes: extrinsic component of external side of plasma membrane [GO:0031232], GO:0031234, extrinsic component of synaptic membrane [GO:0099243] Relationships: is a type of extrinsic component of membrane [GO:0019898]; is part of GO:0005886 Sources: GOC:curators, GOC:dos